RNA transport [GO:0050658] (biological process) Sources: GOC:ai Definition: The directed movement of RNA, ribonucleic acids, into, out of or within a cell, or between cells, by means of some agent such as a transporter or pore. Subtypes: RNA import into nucleus [GO:0006404], GO:0006405, dsRNA transport [GO:0033227], GO:0035927, mRNA transport [GO:0051028], GO:0051029, snRNA transport [GO:0051030], tRNA transport [GO:0051031], miRNA transport [GO:1990428] Relationships: is_a nucleic acid transport [GO:0050657]; is_a GO:0051236